{
  "gene_name": "Phosphoprotein associated with glycosphingolipid-enriched microdomains 1",
  "term_id": "GO:0050868",
  "gene_symbol": "PAG1",
  "term_label": "negative regulation of T cell activation",
  "gene": "UniProtKB:Q9NWQ8"
}